{
  "gene": "UniProtKB:A6BM72",
  "gene_symbol": "MEGF11",
  "term_id": "GO:0005201",
  "term_label": "extracellular matrix structural constituent",
  "gene_name": "Multiple epidermal growth factor-like domains protein 11"
}